{
  "term_id": "GO:0009986",
  "gene_symbol": "LRFN2",
  "gene": "UniProtKB:Q9ULH4",
  "gene_name": "Leucine-rich repeat and fibronectin type-III domain-containing protein 2",
  "term_label": "cell surface"
}